{
  "gene": "UniProtKB:Q9NRP7",
  "gene_symbol": "STK36",
  "gene_name": "Serine_threonine-protein kinase 36",
  "term_id": "UNKNOWN:0001",
  "term_label": "Unknown molecular function"
}